{
  "gene_name": "Vesicular glutamate transporter 2",
  "term_id": "GO:0060076",
  "gene_symbol": "SLC17A6",
  "gene": "UniProtKB:Q9P2U8",
  "term_label": "excitatory synapse"
}